{
  "gene_symbol": "LHX9",
  "gene": "UniProtKB:Q9NQ69",
  "term_label": "regulation of transcription by RNA polymerase II",
  "gene_name": "LIM_homeobox protein Lhx9",
  "term_id": "GO:0006357"
}